L-leucine-2-oxoglutarate transaminase activity [GO:0052654] (MF) Sources: RHEA:18321 Definition: Catalysis of the reaction: 2-oxoglutarate + L-leucine = 4-methyl-2-oxopentanoate + L-glutamatic acid. Relationships: is a type of branched-chain-amino-acid transaminase activity [GO:0004084] Also known as: L-leucine aminotransferase activity